{
  "term_label": "UDP-glucuronate transmembrane transporter activity",
  "gene_symbol": "SLC35D1",
  "gene_name": "Nucleotide sugar transporter SLC35D1",
  "gene": "UniProtKB:Q9NTN3",
  "term_id": "GO:0005461"
}